{
  "gene_symbol": "SFI1",
  "gene": "UniProtKB:A8K8P3",
  "term_label": "Unknown biological process",
  "term_id": "UNKNOWN:0002",
  "gene_name": "Protein SFI1 homolog"
}